regulation of cell differentiation involved in phenotypic switching [GO:1905915] (biological process) References: PMID:25089138 Sources: GOC:BHF, GOC:BHF_miRNA, GOC:TermGenie, GOC:rph, GO_REF:0000058 Relationships: is a type of regulation of cell differentiation [GO:0045595]; regulates cell differentiation involved in phenotypic switching [GO:0090679] Definition: Any process that modulates the frequency, rate or extent of cell differentiation involved in phenotypic switching. Subtypes: negative regulation of cell differentiation involved in phenotypic switching [GO:1905916], positive regulation of cell differentiation involved in phenotypic switching [GO:1905917], regulation of vascular associated smooth muscle cell differentiation involved in phenotypic switching [GO:1905930]